{
  "gene": "UniProtKB:O60603",
  "term_id": "GO:0002224",
  "gene_symbol": "TLR2",
  "term_label": "toll-like receptor signaling pathway",
  "gene_name": "Toll-like receptor 2"
}